Cypridina-luciferin 2-monooxygenase activity [GO:0047712] (molecular function) Also known as: luciferase activity, Cypridina luciferase activity, Cypridina-luciferin:oxygen 2-oxidoreductase (decarboxylating), Cypridina-type luciferase activity, luciferase (Cypridina luciferin) Sources: EC:1.13.12.6, MetaCyc:CYPRIDINA-LUCIFERIN-2-MONOOXYGENASE-RXN Relationships: is a type of oxidoreductase activity, acting on single donors with incorporation of molecular oxygen, incorporation of one atom of oxygen (internal monooxygenases or internal mixed function oxidases) [GO:0016703]; is a type of luciferin monooxygenase activity [GO:0045289] Definition: Catalysis of the reaction: Cypridina luciferin + O2 = oxidized Cypridina luciferin + CO2 + light.